{
  "gene_name": "Hephaestin",
  "term_label": "plasma membrane",
  "gene_symbol": "HEPH",
  "term_id": "GO:0005886",
  "gene": "UniProtKB:Q9BQS7"
}